{
  "gene_name": "C-C motif chemokine 5",
  "term_id": "GO:0048245",
  "gene_symbol": "CCL5",
  "term_label": "eosinophil chemotaxis",
  "gene": "UniProtKB:P13501"
}